{
  "gene": "UniProtKB:P62942",
  "term_label": "sarcoplasmic reticulum membrane",
  "term_id": "GO:0033017",
  "gene_name": "Peptidyl-prolyl cis-trans isomerase FKBP1A",
  "gene_symbol": "FKBP1A"
}